nerve maturation [GO:0021682] (biological process) Definition: A developmental process, independent of morphogenetic (shape) change, that is required for a nerve to attain its fully functional state. Sources: GOC:cls, GOC:dgh, GOC:dph, GOC:jid, GO_REF:0000021 Relationships: is_a anatomical structure maturation [GO:0071695]; is part of nerve development [GO:0021675] Subtypes: cranial nerve maturation [GO:0021605]